{
  "term_id": "UNKNOWN:0003",
  "gene_symbol": "TEX13C",
  "gene": "UniProtKB:A0A0J9YWL9",
  "gene_name": "Putative testis-expressed protein 13C",
  "term_label": "Unknown cellular component"
}